{
  "term_label": "DNA-binding transcription factor activity, RNA polymerase II-specific",
  "gene": "UniProtKB:Q99676",
  "gene_symbol": "ZNF184",
  "term_id": "GO:0000981",
  "gene_name": "Zinc finger protein 184"
}